positive regulation of AV node cell action potential [GO:1903951] (biological process) Also known as: positive regulation of AV node cardiac muscle cell action potential, positive regulation of atrioventricular node cardiac muscle cell action potential, up regulation of AV node cardiac muscle cell action potential, up regulation of AV node cell action potential, up regulation of atrioventricular node cardiac muscle cell action potential, up-regulation of AV node cardiac muscle cell action potential, up-regulation of AV node cell action potential, up-regulation of atrioventricular node cardiac muscle cell action potential, upregulation of AV node cardiac muscle cell action potential, upregulation of AV node cell action potential, upregulation of atrioventricular node cardiac muscle cell action potential, activation of AV node cardiac muscle cell action potential, activation of AV node cell action potential, activation of atrioventricular node cardiac muscle cell action potential Definition: Any process that activates or increases the frequency, rate or extent of AV node cell action potential. References: PMID:25281747 Sources: GOC:BHF, GOC:TermGenie, GOC:mtg_cardiac_conduct_nov11, GOC:nc, GO_REF:0000058 Relationships: is a type of positive regulation of action potential [GO:0045760]; is a type of GO:0098904; positively regulates AV node cell action potential [GO:0086016]